{
  "term_id": "GO:0019731",
  "gene": "UniProtKB:P57053",
  "gene_symbol": "H2BC12L",
  "term_label": "antibacterial humoral response",
  "gene_name": "Histone H2B type F-S"
}